{
  "gene_symbol": "EXPH5",
  "term_id": "GO:0050714",
  "gene_name": "Exophilin-5",
  "term_label": "positive regulation of protein secretion",
  "gene": "UniProtKB:Q8NEV8"
}